{
  "term_id": "GO:0003352",
  "gene_name": "Dynein regulatory complex protein 1",
  "term_label": "regulation of cilium movement",
  "gene": "UniProtKB:Q96MC2",
  "gene_symbol": "DRC1"
}